{
  "term_id": "GO:0005634",
  "gene": "UniProtKB:Q96DN6",
  "gene_name": "Methyl-CpG-binding domain protein 6",
  "gene_symbol": "MBD6",
  "term_label": "nucleus"
}